{
  "gene_name": "Vitamin D3 receptor",
  "term_label": "vitamin D response element binding",
  "gene": "UniProtKB:P11473",
  "term_id": "GO:0070644",
  "gene_symbol": "VDR"
}